{
  "gene": "UniProtKB:P07327",
  "gene_name": "Alcohol dehydrogenase 1A",
  "term_id": "GO:0042573",
  "gene_symbol": "ADH1A",
  "term_label": "retinoic acid metabolic process"
}